{
  "gene": "UniProtKB:Q9UBD6",
  "gene_name": "Ammonium transporter Rh type C",
  "term_label": "ammonium transmembrane transport",
  "term_id": "GO:0072488",
  "gene_symbol": "RHCG"
}